{
  "gene_name": "Apolipoprotein C-II",
  "gene": "UniProtKB:P02655",
  "gene_symbol": "APOC2",
  "term_id": "GO:0042159",
  "term_label": "lipoprotein catabolic process"
}